{
  "term_id": "UNKNOWN:0001",
  "gene": "UniProtKB:Q8TCH9",
  "term_label": "Unknown molecular function",
  "gene_symbol": "Q8TCH9",
  "gene_name": "Putative uncharacterized protein FLJ23865"
}